{
  "gene": "UniProtKB:Q86YF9",
  "term_id": "GO:0140311",
  "gene_symbol": "DZIP1",
  "gene_name": "Cilium assembly protein DZIP1",
  "term_label": "protein sequestering activity"
}